hormone biosynthetic process [GO:0042446] (biological process) Relationships: is a type of biosynthetic process [GO:0009058]; is_a hormone metabolic process [GO:0042445] Sources: GOC:jl Definition: The chemical reactions and pathways resulting in the formation of any hormone, naturally occurring substances secreted by specialized cells that affects the metabolism or behavior of other cells possessing functional receptors for the hormone. Regulation: negatively regulated by negative regulation of hormone biosynthetic process [GO:0032353]; regulated by regulation of hormone biosynthetic process [GO:0046885]; positively regulated by positive regulation of hormone biosynthetic process [GO:0046886] Subtypes: C21-steroid hormone biosynthetic process [GO:0006700], androgen biosynthetic process [GO:0006702], estrogen biosynthetic process [GO:0006703], mineralocorticoid biosynthetic process [GO:0006705], juvenile hormone biosynthetic process [GO:0006718], cytokinin biosynthetic process [GO:0009691], auxin biosynthetic process [GO:0009851], melatonin biosynthetic process [GO:0030187], pheromone biosynthetic process [GO:0042811], ecdysteroid biosynthetic process [GO:0045456] Also known as: hormone anabolism, hormone biosynthesis, hormone formation, hormone synthesis